{
  "term_label": "protein processing",
  "gene_name": "Cysteine protease ATG4D",
  "gene_symbol": "ATG4D",
  "gene": "UniProtKB:Q86TL0",
  "term_id": "GO:0016485"
}